{
  "gene_name": "Gamma-secretase subunit APH-1B",
  "term_id": "GO:0016485",
  "gene_symbol": "APH1B",
  "term_label": "protein processing",
  "gene": "UniProtKB:Q8WW43"
}